{
  "gene_name": "FHF complex subunit HOOK-interacting protein 1B",
  "gene_symbol": "FHIP1B",
  "term_id": "GO:0045022",
  "term_label": "early endosome to late endosome transport",
  "gene": "UniProtKB:Q8N612"
}